{
  "term_label": "NuA4 histone acetyltransferase complex",
  "term_id": "GO:0035267",
  "gene_name": "Male-specific lethal 3 homolog",
  "gene_symbol": "MSL3",
  "gene": "UniProtKB:Q8N5Y2"
}